meiotic joint molecule formation [GO:0000709] (biological process) Regulation: regulated by regulation of meiotic joint molecule formation [GO:0010946]; negatively regulated by negative regulation of meiotic joint molecule formation [GO:0010947] Relationships: is a type of meiotic cell cycle process [GO:1903046]; BFO_0000050 reciprocal meiotic recombination [GO:0007131] References: PMID:8521495 Sources: GOC:elh Definition: The conversion of the paired broken DNA and homologous duplex DNA into a four-stranded branched intermediate, known as a joint molecule, formed during meiotic recombination. These joint molecules contain Holliday junctions on either side of heteroduplex DNA.